{
  "term_label": "Unknown molecular function",
  "gene_symbol": "LINC00477",
  "term_id": "UNKNOWN:0001",
  "gene": "UniProtKB:Q96M19",
  "gene_name": "Putative transmembrane protein encoded by LINC00477"
}